{
  "term_id": "UNKNOWN:0003",
  "term_label": "Unknown cellular component",
  "gene_symbol": "KDM1B",
  "gene_name": "Lysine-specific histone demethylase 2",
  "gene": "UniProtKB:Q8NB78"
}